{
  "term_label": "Unknown biological process",
  "gene_name": "Sperm-associated antigen 11A",
  "term_id": "UNKNOWN:0002",
  "gene_symbol": "SPAG11A",
  "gene": "UniProtKB:Q6PDA7"
}